{
  "term_label": "regulation of transcription by RNA polymerase II",
  "gene_symbol": "ZNF224",
  "gene": "UniProtKB:Q9NZL3",
  "term_id": "GO:0006357",
  "gene_name": "Zinc finger protein 224"
}